4-hydroxybutyrate receptor activity [GO:0062124] (molecular function) Definition: Combining with 4-hydroxybutyrte to initiate a change in cell activity. Relationships: is_a signaling receptor activity [GO:0038023] Also known as: gamma-hydroxybutyrate receptor activity References: PMID:17197387